{
  "term_id": "GO:0008017",
  "gene": "UniProtKB:Q96SN8",
  "gene_symbol": "CDK5RAP2",
  "term_label": "microtubule binding",
  "gene_name": "CDK5 regulatory subunit-associated protein 2"
}